{
  "gene": "UniProtKB:Q9BWF3",
  "term_label": "nuclear speck",
  "gene_name": "RNA-binding protein 4",
  "gene_symbol": "RBM4",
  "term_id": "GO:0016607"
}